{
  "term_id": "UNKNOWN:0003",
  "gene_symbol": "CTXN1",
  "gene": "UniProtKB:P60606",
  "gene_name": "Cortexin-1",
  "term_label": "Unknown cellular component"
}